{
  "gene_name": "DNA repair protein XRCC2",
  "gene_symbol": "XRCC2",
  "gene": "UniProtKB:O43543",
  "term_label": "DNA strand invasion",
  "term_id": "GO:0042148"
}